{
  "term_id": "GO:0005634",
  "gene": "UniProtKB:Q9H3R5",
  "term_label": "nucleus",
  "gene_symbol": "CENPH",
  "gene_name": "Centromere protein H"
}